{
  "gene": "UniProtKB:P01611",
  "term_label": "immune response",
  "gene_symbol": "IGKV1D-12",
  "term_id": "GO:0006955",
  "gene_name": "Immunoglobulin kappa variable 1D-12"
}